{
  "gene_name": "Sushi domain-containing protein 2",
  "term_label": "plasma membrane",
  "term_id": "GO:0005886",
  "gene_symbol": "SUSD2",
  "gene": "UniProtKB:Q9UGT4"
}